{
  "gene_symbol": "DOK1",
  "gene": "UniProtKB:Q99704",
  "gene_name": "Docking protein 1",
  "term_label": "Unknown cellular component",
  "term_id": "UNKNOWN:0003"
}